{
  "gene_symbol": "MMP1",
  "gene_name": "Interstitial collagenase",
  "gene": "UniProtKB:P03956",
  "term_id": "GO:0030574",
  "term_label": "collagen catabolic process"
}